regulation of netrin-activated signaling pathway [GO:1902841] (biological process) References: PMID:24004945 Sources: GOC:TermGenie, GOC:kmv, GO_REF:0000058 Relationships: is a type of regulation of signal transduction [GO:0009966]; regulates GO:0038007 Subtypes: negative regulation of netrin-activated signaling pathway [GO:1902842], positive regulation of netrin-activated signaling pathway [GO:1902843] Also known as: regulation of netrin signaling pathway, regulation of netrin-activated signal transduction pathway, regulation of netrin-activated signalling pathway, regulation of netrin-mediated signaling pathway Definition: Any process that modulates the frequency, rate or extent of netrin-activated signaling pathway.